tricyclic triterpenoid catabolic process [GO:0010684] (biological process) Also known as: tricyclic triterpenoid catabolism Definition: The chemical reactions and pathways resulting in the breakdown of tricyclic triterpenoid compounds, terpenoids with six isoprene units and 3 rings. Sources: GOC:tair_curators Relationships: is a type of triterpenoid catabolic process [GO:0016105]